{
  "gene_symbol": "DCTPP1",
  "gene": "UniProtKB:Q9H773",
  "term_id": "GO:0006253",
  "term_label": "dCTP catabolic process",
  "gene_name": "dCTP pyrophosphatase 1"
}